{
  "gene_name": "Sterile alpha motif domain-containing protein 11",
  "gene": "UniProtKB:Q96NU1",
  "term_id": "GO:0005634",
  "gene_symbol": "SAMD11",
  "term_label": "nucleus"
}